{
  "term_id": "GO:0005739",
  "gene_symbol": "PRDX3",
  "term_label": "mitochondrion",
  "gene": "UniProtKB:P30048",
  "gene_name": "Thioredoxin-dependent peroxide reductase, mitochondrial"
}